selenodiglutathione-disulfide reductase (NADPH) activity [GO:0098622] (molecular function) Also known as: selenodiglutathione-disulfide reductase activity, selenodiglutathione-disulfide reductase (NADP) activity Relationships: is a type of GO:0015036; is a type of GO:0016668 Definition: Catalysis of the reaction: H+ + selenodiglutathione + NADPH = gluthathioselenol + glutathione + NADP+. References: PMID:1569062 Sources: RHEA:34927